positive regulation of epithelial cell proliferation involved in lung bud dilation [GO:0060504] (biological process) Relationships: is a type of GO:0048639; is a type of positive regulation of epithelial cell proliferation involved in lung morphogenesis [GO:0060501]; is_a positive regulation of branching involved in lung morphogenesis [GO:0061047]; positively regulates epithelial cell proliferation involved in lung bud dilation [GO:0060505] Sources: GOC:dph Definition: Any process that increases the rate or frequency of epithelial cell proliferation that results in the lung bud increasing in size radially.